response to dsRNA [GO:0043331] (biological process) Definition: Any process that results in a change in state or activity of a cell or an organism (in terms of movement, secretion, enzyme production, gene expression, etc.) as a result of a double-stranded RNA stimulus. Sources: GOC:jl Also known as: response to double-stranded RNA Subtypes: GO:0043330, cellular response to dsRNA [GO:0071359] Relationships: is a type of response to nitrogen compound [GO:1901698]